{
  "gene_name": "Zinc finger homeobox protein 2",
  "term_label": "RNA polymerase II cis-regulatory region sequence-specific DNA binding",
  "gene_symbol": "ZFHX2",
  "term_id": "GO:0000978",
  "gene": "UniProtKB:Q9C0A1"
}